instrumental aggressive behavior [GO:0002126] (biological process) Relationships: is a type of GO:0002118 Sources: GOC:hjd Also known as: instrumental aggression Definition: Aggressive behavior directed towards obtaining some goal, considered to be a learned response to a situation.